{
  "gene": "UniProtKB:Q9BRC7",
  "term_label": "phosphatidylinositol-4,5-bisphosphate phospholipase C activity",
  "gene_symbol": "PLCD4",
  "gene_name": "1-phosphatidylinositol 4,5-bisphosphate phosphodiesterase delta-4",
  "term_id": "GO:0004435"
}